trigeminal ganglion structural organization [GO:0061563] (biological process) Definition: The process that contributes to creating the structural organization of the trigeminal ganglion This process pertains to the physical shaping of a rudimentary structure. Relationships: is a type of cranial ganglion structural organization [GO:0061562]; is part of trigeminal nerve structural organization [GO:0021637]; is part of GO:0061556 Also known as: trigeminal ganglia organization Sources: GOC:dph